{
  "term_label": "RNA polymerase II transcription regulatory region sequence-specific DNA binding",
  "gene_symbol": "PURA",
  "gene_name": "Transcriptional activator protein Pur-alpha",
  "term_id": "GO:0000977",
  "gene": "UniProtKB:Q00577"
}